{
  "term_id": "UNKNOWN:0003",
  "term_label": "Unknown cellular component",
  "gene": "UniProtKB:A1L162",
  "gene_symbol": "ERICH2",
  "gene_name": "Glutamate-rich protein 2"
}